canonical Wnt signaling pathway involved in negative regulation of apoptotic process [GO:0044336] (biological process) Relationships: is a type of GO:0060070; is part of GO:0043066 Also known as: canonical Wnt receptor signaling pathway involved in negative regulation of apoptotic process, canonical Wnt receptor signalling pathway involved in negative regulation of apoptosis, canonical Wnt receptor signaling pathway involved in negative regulation of apoptosis Sources: GOC:BHF, GOC:jl, GOC:mtg_apoptosis Definition: The series of molecular signals initiated by binding of a Wnt protein to a frizzled family receptor on the surface of the target cell, followed by propagation of the signal via beta-catenin, and ending with a change in transcription of target genes involved in the negative regulation of apoptotic process.